{
  "term_id": "GO:0009897",
  "gene_name": "Placenta-expressed transcript 1 protein",
  "term_label": "external side of plasma membrane",
  "gene_symbol": "PLET1",
  "gene": "UniProtKB:Q6UQ28"
}